{
  "term_label": "nucleus",
  "gene_symbol": "UGDH",
  "term_id": "GO:0005634",
  "gene_name": "UDP-glucose 6-dehydrogenase",
  "gene": "UniProtKB:O60701"
}